{
  "gene_name": "Phosducin-like protein 3",
  "term_id": "GO:0010628",
  "gene_symbol": "PDCL3",
  "gene": "UniProtKB:Q9H2J4",
  "term_label": "positive regulation of gene expression"
}